{
  "term_id": "UNKNOWN:0003",
  "gene_name": "F-box only protein 47",
  "gene_symbol": "FBXO47",
  "term_label": "Unknown cellular component",
  "gene": "UniProtKB:Q5MNV8"
}